{
  "gene_symbol": "HNF4A",
  "term_label": "positive regulation of transcription by RNA polymerase II",
  "gene": "UniProtKB:P41235",
  "term_id": "GO:0045944",
  "gene_name": "Hepatocyte nuclear factor 4-alpha"
}